epithelial cell differentiation involved in kidney development [GO:0035850] (biological process) References: PMID:16216236 Sources: GOC:bf, GOC:mtg_kidney_jan10, GOC:yaf Definition: The process in which relatively unspecialized cells acquire specialized structural and/or functional features of an epithelial cell that characterize the cells of the kidney as it progresses from its formation to the mature state. Relationships: is a type of epithelial cell differentiation [GO:0030855]; is a type of cell differentiation involved in kidney development [GO:0061005] Regulation: regulated by regulation of epithelial cell differentiation involved in kidney development [GO:2000696]; negatively regulated by GO:2000697; positively regulated by positive regulation of epithelial cell differentiation involved in kidney development [GO:2000698] Subtypes: mesenchymal to epithelial transition involved in metanephros morphogenesis [GO:0003337], GO:0061261, glomerular mesangial cell differentiation [GO:0072008], mesenchymal to epithelial transition involved in renal vesicle formation [GO:0072036], nephron tubule epithelial cell differentiation [GO:0072160], glomerular epithelial cell differentiation [GO:0072311]